{
  "gene_symbol": "SAR1A",
  "term_label": "endoplasmic reticulum to Golgi vesicle-mediated transport",
  "term_id": "GO:0006888",
  "gene": "UniProtKB:Q9NR31",
  "gene_name": "GTP-binding protein SAR1a"
}